{
  "term_label": "voltage-gated sodium channel complex",
  "gene_name": "Sodium channel protein type 1 subunit alpha",
  "term_id": "GO:0001518",
  "gene_symbol": "SCN1A",
  "gene": "UniProtKB:P35498"
}